lysosomal lumen pH elevation [GO:0035752] (biological process) Also known as: lysosome pH elevation Relationships: is a type of regulation of lysosomal lumen pH [GO:0035751]; is a type of intracellular pH elevation [GO:0051454] Definition: Any process that increases the pH of the lysosomal lumen, measured by the concentration of the hydrogen ion. Sources: GOC:bf, GOC:rph